{
  "term_label": "nucleus",
  "gene_name": "Nuclear RNA export factor 2",
  "gene_symbol": "NXF2B",
  "gene": "UniProtKB:Q9GZY0",
  "term_id": "GO:0005634"
}